{
  "gene": "UniProtKB:Q9Y5Z0",
  "term_id": "GO:0005802",
  "gene_symbol": "BACE2",
  "gene_name": "Beta-secretase 2",
  "term_label": "trans-Golgi network"
}